{
  "gene_name": "Deoxynucleotidyltransferase terminal-interacting protein 1",
  "gene_symbol": "DNTTIP1",
  "term_label": "nucleosome binding",
  "term_id": "GO:0031491",
  "gene": "UniProtKB:Q9H147"
}